proximal convoluted tubule segment 1 cell differentiation [GO:0072062] (biological process) Definition: The process in which relatively unspecialized cells acquire specialized structural and/or functional features that characterize the S1 cells of the kidney as it progresses from its formation to the mature state. Sources: GOC:bf, GOC:mtg_kidney_jan10 Also known as: S1 cell differentiation Relationships: is a type of cell differentiation involved in kidney development [GO:0061005]; is part of proximal convoluted tubule segment 1 development [GO:0072031]